{
  "gene_symbol": "OR5T1",
  "term_id": "GO:0007608",
  "term_label": "sensory perception of smell",
  "gene_name": "Olfactory receptor 5T1",
  "gene": "UniProtKB:Q8NG75"
}